{
  "gene_name": "Serine_threonine-protein phosphatase 2A catalytic subunit alpha isoform",
  "gene_symbol": "PPP2CA",
  "term_id": "GO:0000278",
  "gene": "UniProtKB:P67775",
  "term_label": "mitotic cell cycle"
}